{
  "term_label": "cell motility",
  "gene_name": "Actin, cytoplasmic 1",
  "gene": "UniProtKB:P60709",
  "term_id": "GO:0048870",
  "gene_symbol": "ACTB"
}